{
  "term_label": "presynaptic membrane",
  "gene_symbol": "CADM3",
  "gene_name": "Cell adhesion molecule 3",
  "term_id": "GO:0042734",
  "gene": "UniProtKB:Q8N126"
}